{
  "term_label": "Unknown molecular function",
  "gene_name": "Up-regulator of cell proliferation",
  "gene_symbol": "URGCP",
  "gene": "UniProtKB:Q8TCY9",
  "term_id": "UNKNOWN:0001"
}